{
  "gene": "UniProtKB:O15055",
  "term_id": "GO:0032922",
  "gene_name": "Period circadian protein homolog 2",
  "term_label": "circadian regulation of gene expression",
  "gene_symbol": "PER2"
}